{
  "term_id": "GO:0000139",
  "gene_symbol": "ST6GALNAC1",
  "gene": "UniProtKB:Q9NSC7",
  "term_label": "Golgi membrane",
  "gene_name": "Alpha-N-acetylgalactosaminide alpha-2,6-sialyltransferase 1"
}